{
  "gene_name": "Protein myomaker",
  "term_label": "Unknown molecular function",
  "term_id": "UNKNOWN:0001",
  "gene_symbol": "MYMK",
  "gene": "UniProtKB:A6NI61"
}